{
  "term_label": "Unknown biological process",
  "gene_name": "Late cornified envelope protein 6A",
  "gene_symbol": "LCE6A",
  "gene": "UniProtKB:A0A183",
  "term_id": "UNKNOWN:0002"
}